positive regulation of mRNA catabolic process [GO:0061014] (biological process) Also known as: positive regulation of mRNA decay Definition: Any process that increases the rate, frequency, or extent of a mRNA catabolic process, the chemical reactions and pathways resulting in the breakdown of RNA, ribonucleic acid, one of the two main type of nucleic acid, consisting of a long, unbranched macromolecule formed from ribonucleotides joined in 3',5'-phosphodiester linkage. Subtypes: GO:0060213, mRNA destabilization [GO:0061157], positive regulation of nuclear mRNA surveillance of meiosis-specific transcripts [GO:0120272], GO:1900153, positive regulation of deadenylation-independent decapping of nuclear-transcribed mRNA [GO:1901835], positive regulation of mitochondrial mRNA catabolic process [GO:1905639], negative regulation of 3'-UTR-mediated mRNA stabilization [GO:1905869], positive regulation of nuclear-transcribed mRNA catabolic process, nonsense-mediated decay [GO:2000624] Relationships: is a type of positive regulation of catabolic process [GO:0009896]; is a type of regulation of mRNA catabolic process [GO:0061013]; is a type of positive regulation of mRNA metabolic process [GO:1903313]; positively regulates GO:0006402 Sources: GOC:ascb_2009, GOC:dph, GOC:tb